chlorophyll(ide) b reductase activity [GO:0034256] (molecular function) Relationships: is a type of oxidoreductase activity, acting on the CH-OH group of donors, NAD or NADP as acceptor [GO:0016616] Definition: Catalysis of the reaction: 71-hydroxychlorophyll(ide) a + NAD(P)+ = chlorophyll(ide) b + NAD(P)H + H+. Sources: EC:1.1.1.294, MetaCyc:RXN-7678 Also known as: Chl b reductase activity, chlorophyll b reductase activity, chlorophyllide b reductase activity